{
  "term_id": "GO:0045109",
  "gene_symbol": "VIM",
  "gene": "UniProtKB:P08670",
  "term_label": "intermediate filament organization",
  "gene_name": "Vimentin"
}